{
  "term_label": "T cell receptor signaling pathway",
  "gene_symbol": "DENND1B",
  "gene_name": "DENN domain-containing protein 1B",
  "gene": "UniProtKB:Q6P3S1",
  "term_id": "GO:0050852"
}